{
  "gene_symbol": "VPS37B",
  "term_id": "GO:0006612",
  "gene_name": "Vacuolar protein sorting-associated protein 37B",
  "term_label": "protein targeting to membrane",
  "gene": "UniProtKB:Q9H9H4"
}